compound eye morphogenesis [GO:0001745] (BP) Also known as: insect-type retina morphogenesis Definition: The morphogenetic process in which the anatomical structures of the compound eye are generated and organized. The adult compound eye is a precise assembly of 700-800 ommatidia. Each ommatidium is composed of 20 cells, identified by cell type and position. An example of compound eye morphogenesis is found in Drosophila melanogaster. Relationships: is a type of eye morphogenesis [GO:0048592]; is part of GO:0048749 Sources: GOC:dph, GOC:mtg_sensu